cellular detoxification of hydrogen peroxide [GO:0061692] (biological process) Definition: Any process that reduces or removes the toxicity of hydrogen peroxide in a cell. These include transport of hydrogen peroxide away from sensitive areas and to compartments or complexes whose purpose is sequestration. Sources: GOC:dph, GOC:vw Relationships: is a type of detoxification of hydrogen peroxide [GO:0061691]; is a type of cellular oxidant detoxification [GO:0098869]; is part of cellular response to hydrogen peroxide [GO:0070301]